{
  "gene": "UniProtKB:O94760",
  "gene_symbol": "DDAH1",
  "term_id": "GO:0016403",
  "gene_name": "N(G),N(G)-dimethylarginine dimethylaminohydrolase 1",
  "term_label": "dimethylargininase activity"
}